{
  "term_id": "UNKNOWN:0003",
  "gene_symbol": "TEX13A",
  "gene_name": "Testis-expressed protein 13A",
  "gene": "UniProtKB:Q9BXU3",
  "term_label": "Unknown cellular component"
}